oxidoreductase activity, acting on hydrogen as donor, cytochrome as acceptor [GO:0016697] (MF) Relationships: is a type of oxidoreductase activity, acting on hydrogen as donor [GO:0016695] Definition: Catalysis of an oxidation-reduction (redox) reaction in which hydrogen acts as an electron donor and reduces a cytochrome. Sources: GOC:jl Subtypes: GO:0047806